anthranilate 3-monooxygenase (deaminating) activity [GO:0018672] (molecular function) Relationships: is a type of oxidoreductase activity, acting on paired donors, with incorporation or reduction of molecular oxygen, NAD(P)H as one donor, and incorporation of one atom of oxygen [GO:0016709] Sources: EC:1.14.13.35, RHEA:21236 Also known as: anthranilate hydroxylase activity, anthranilate hydroxylase (deaminating) activity, anthranilate 2,3-dioxygenase (deaminating), anthranilate 2,3-hydroxylase (deaminating) activity, anthranilate,NADPH:oxygen oxidoreductase (3-hydroxylating, deaminating) Definition: Catalysis of the reaction: anthranilate + 2 H+ + NADPH + O2 = 2,3-dihydroxybenzoate + NADP+ + NH4.